nematocyst [GO:0042151] (cellular component) Definition: An organelle found in cnidoblast (nematoblast) cells. When matured, these stinging organelles store toxins and can deliver them when the cnidocil (a short extension of the cnidocyst) is stimulated by a prey or another stimulus. Sources: DOI:10.1139/z02-135, GOC:jl Relationships: is a type of intracellular membraneless organelle [GO:0043232]; is part of cell cortex [GO:0005938] Also known as: cnidocyst